{
  "gene_name": "Keratin-associated protein 13-4",
  "term_label": "Unknown biological process",
  "gene": "UniProtKB:Q3LI77",
  "gene_symbol": "KRTAP13-4",
  "term_id": "UNKNOWN:0002"
}